{
  "gene_name": "Uncharacterized protein GAS8-AS1",
  "term_id": "UNKNOWN:0001",
  "gene": "UniProtKB:O95177",
  "term_label": "Unknown molecular function",
  "gene_symbol": "GAS8-AS1"
}